{
  "term_id": "GO:0031267",
  "gene": "UniProtKB:Q9NQG7",
  "term_label": "small GTPase binding",
  "gene_symbol": "HPS4",
  "gene_name": "BLOC-3 complex member HPS4"
}